{
  "term_label": "regulation of protein stability",
  "gene": "UniProtKB:Q14694",
  "gene_name": "Ubiquitin carboxyl-terminal hydrolase 10",
  "term_id": "GO:0031647",
  "gene_symbol": "USP10"
}